{
  "term_id": "GO:0005739",
  "gene_symbol": "TMEM65",
  "gene": "UniProtKB:Q6PI78",
  "gene_name": "Transmembrane protein 65",
  "term_label": "mitochondrion"
}